{
  "gene_symbol": "MFN2",
  "term_label": "GTPase activity",
  "gene_name": "Mitofusin-2",
  "term_id": "GO:0003924",
  "gene": "UniProtKB:O95140"
}